{
  "gene_name": "Suppressor of cytokine signaling 6",
  "gene_symbol": "SOCS6",
  "gene": "UniProtKB:O14544",
  "term_id": "UNKNOWN:0003",
  "term_label": "Unknown cellular component"
}